non-proteinogenic amino acid catabolic process [GO:0170044] (biological process) Sources: GOC:ew Subtypes: L-ornithine catabolic process [GO:0006593], gamma-aminobutyric acid catabolic process [GO:0009450], L-citrulline catabolic process [GO:0019241], trans-4-hydroxy-L-proline catabolic process [GO:0019470], D-amino acid catabolic process [GO:0019478], beta-alanine catabolic process [GO:0019484], L-proline betaine catabolic process [GO:0019504], S-adenosylhomocysteine catabolic process [GO:0019510], GO:0034269, 1-aminocyclopropane-1-carboxylate catabolic process [GO:0042217], homocysteine catabolic process [GO:0043418], phosphoarginine catabolic process [GO:0046313], hydroxylysine catabolic process [GO:0046948], L-kynurenine catabolic process [GO:0097053], sarcosine catabolic process [GO:1901053], 3-cyano-L-alanine catabolic process [GO:1903559], N(omega)-methyl-L-arginine catabolic process [GO:2001297], N(omega),N(omega)-dimethyl-L-arginine catabolic process [GO:2001299] Definition: The chemical reactions and pathways resulting in the breakdown of non-proteinogenic amino acids. Also known as: non-proteinogenic amino acid breakdown, non-proteinogenic amino acid catabolism, non-proteinogenic amino acid degradation Relationships: is a type of carboxylic acid catabolic process [GO:0046395]; is a type of GO:0170041